bicellular tight junction [GO:0005923] (cellular component) Sources: GOC:mah, ISBN:0815332181 Also known as: zonula occludens Relationships: is a type of tight junction [GO:0070160]; is part of GO:0043296 Subtypes: host-symbiont bicellular tight junction [GO:0044647] Definition: An occluding cell-cell junction that is composed of a branching network of sealing strands that completely encircles the apical end of each cell in an epithelial sheet; the outer leaflets of the two interacting plasma membranes are seen to be tightly apposed where sealing strands are present. Each sealing strand is composed of a long row of transmembrane adhesion proteins embedded in each of the two interacting plasma membranes.